{
  "gene_name": "Cancer_testis antigen family 45 member A2",
  "gene": "UniProtKB:Q5DJT8",
  "gene_symbol": "CT45A2",
  "term_id": "UNKNOWN:0002",
  "term_label": "Unknown biological process"
}